{
  "term_id": "GO:0016020",
  "gene": "UniProtKB:Q9UBS9",
  "gene_symbol": "SUCO",
  "term_label": "membrane",
  "gene_name": "SUN domain-containing ossification factor"
}